{
  "gene_name": "Solute carrier family 28 member 3",
  "term_label": "pyrimidine- and adenosine-specific:sodium symporter activity",
  "gene": "UniProtKB:Q9HAS3",
  "gene_symbol": "SLC28A3",
  "term_id": "GO:0015389"
}